{
  "term_id": "GO:0000978",
  "gene": "UniProtKB:Q96ND8",
  "term_label": "RNA polymerase II cis-regulatory region sequence-specific DNA binding",
  "gene_symbol": "ZNF583",
  "gene_name": "Zinc finger protein 583"
}